{
  "term_label": "Unknown biological process",
  "gene": "UniProtKB:B3EWF7",
  "term_id": "UNKNOWN:0002",
  "gene_symbol": "EPM2A",
  "gene_name": "Laforin, isoform 9"
}